{
  "gene": "UniProtKB:Q9NQW6",
  "term_id": "GO:0000915",
  "gene_symbol": "ANLN",
  "term_label": "actomyosin contractile ring assembly",
  "gene_name": "Anillin"
}